{
  "term_id": "GO:0016477",
  "term_label": "cell migration",
  "gene_name": "Breast cancer anti-estrogen resistance protein 1",
  "gene_symbol": "BCAR1",
  "gene": "UniProtKB:P56945"
}